{
  "term_id": "GO:0007076",
  "term_label": "mitotic chromosome condensation",
  "gene": "UniProtKB:Q15021",
  "gene_name": "Condensin complex subunit 1",
  "gene_symbol": "NCAPD2"
}